{
  "gene_symbol": "RALB",
  "term_id": "GO:0003924",
  "term_label": "GTPase activity",
  "gene": "UniProtKB:P11234",
  "gene_name": "Ras-related protein Ral-B"
}